regulation of synaptic metaplasticity [GO:0031916] (biological process) Relationships: is a type of regulation of synaptic plasticity [GO:0048167] Subtypes: negative regulation of synaptic metaplasticity [GO:0031917], positive regulation of synaptic metaplasticity [GO:0031918] Definition: A process that modulates synaptic metaplasticity. Metaplasticity is a higher-order form of plasticity and is manifest as a change in the ability to induce subsequent synaptic plasticity that is the ability of synapses to change as circumstances require. References: PMID:8658594 Sources: GOC:mah